{
  "gene_name": "Ras-related protein Rab-19",
  "term_label": "GTPase activity",
  "gene": "UniProtKB:A4D1S5",
  "gene_symbol": "RAB19",
  "term_id": "GO:0003924"
}